DNA conformation change [GO:0071103] (biological process) Subtypes: DNA topological change [GO:0006265], DNA geometric change [GO:0032392] Definition: A cellular process that results in a change in the spatial configuration of a DNA molecule. A conformation change can bend DNA, or alter the, twist, writhe, or linking number of a DNA molecule. Also known as: DNA conformation modification Sources: GOC:mah Relationships: is a type of GO:0051276